{
  "term_id": "GO:0006325",
  "term_label": "chromatin organization",
  "gene": "UniProtKB:Q2TAK8",
  "gene_name": "PWWP domain-containing DNA repair factor 3A",
  "gene_symbol": "PWWP3A"
}